{
  "gene_name": "Protein Hook homolog 2",
  "term_id": "GO:0051959",
  "gene_symbol": "HOOK2",
  "gene": "UniProtKB:Q96ED9",
  "term_label": "dynein light intermediate chain binding"
}